{
  "gene": "UniProtKB:A6NC51",
  "gene_name": "Modulator of macroautophagy TMEM150B",
  "gene_symbol": "TMEM150B",
  "term_id": "UNKNOWN:0002",
  "term_label": "Unknown biological process"
}